determination of ventral identity [GO:0048264] (BP) Relationships: is a type of dorsal/ventral pattern formation [GO:0009953]; is part of determination of dorsal/ventral asymmetry [GO:0048262] Sources: GOC:dph, GOC:isa_complete, GOC:jid Definition: The regionalization process that results in the determination of the identity of part of an organism or organ where those parts are of the type that occur in the ventral region. Identity is considered to be the aggregate of characteristics by which a structure is recognized. Also known as: determination of abaxial identity